{
  "gene_name": "Zinc finger protein 706",
  "gene_symbol": "ZNF706",
  "term_id": "UNKNOWN:0003",
  "term_label": "Unknown cellular component",
  "gene": "UniProtKB:Q9Y5V0"
}